{
  "gene_symbol": "CREBRF",
  "term_id": "GO:0005634",
  "term_label": "nucleus",
  "gene_name": "CREB3 regulatory factor",
  "gene": "UniProtKB:Q8IUR6"
}